{
  "term_id": "GO:0000977",
  "gene_name": "Achaete-scute homolog 4",
  "term_label": "RNA polymerase II transcription regulatory region sequence-specific DNA binding",
  "gene": "UniProtKB:Q6XD76",
  "gene_symbol": "ASCL4"
}